{
  "term_id": "GO:0006559",
  "gene_name": "Maleylacetoacetate isomerase",
  "term_label": "L-phenylalanine catabolic process",
  "gene": "UniProtKB:O43708",
  "gene_symbol": "GSTZ1"
}